{
  "gene": "UniProtKB:Q7L7L0",
  "gene_symbol": "H2AC25",
  "term_label": "structural constituent of chromatin",
  "gene_name": "Histone H2A type 3",
  "term_id": "GO:0030527"
}